positive regulation of membrane repolarization during ventricular cardiac muscle cell action potential [GO:1905026] (biological process) Definition: Any process that activates or increases the frequency, rate or extent of membrane repolarization during ventricular cardiac muscle cell action potential. References: PMID:19893015 Sources: GOC:BHF, GOC:BHF_miRNA, GOC:TermGenie, GOC:mtg_cardiac_conduct_nov11, GOC:rph Relationships: is a type of regulation of membrane repolarization during ventricular cardiac muscle cell action potential [GO:1905024]; is a type of GO:1905033; positively regulates GO:0098915 Also known as: up regulation of membrane repolarization during ventricular cardiac muscle cell action potential, up-regulation of membrane repolarization during ventricular cardiac muscle cell action potential, upregulation of membrane repolarization during ventricular cardiac muscle cell action potential, activation of membrane repolarization during ventricular cardiac muscle cell action potential, activation of electrocardiogram T wave, activation of regulation of ventricular cardiac muscle repolarization, activation of ventricular repolarization, positive regulation of electrocardiogram T wave, positive regulation of regulation of ventricular cardiac muscle repolarization, positive regulation of ventricular repolarization, up regulation of electrocardiogram T wave, up regulation of regulation of ventricular cardiac muscle repolarization, up regulation of ventricular repolarization, up-regulation of electrocardiogram T wave, up-regulation of regulation of ventricular cardiac muscle repolarization, up-regulation of ventricular repolarization, upregulation of electrocardiogram T wave, upregulation of regulation of ventricular cardiac muscle repolarization, upregulation of ventricular repolarization